{
  "gene_name": "Histone H2A type 1-J",
  "gene_symbol": "H2AC14",
  "term_label": "nucleus",
  "term_id": "GO:0005634",
  "gene": "UniProtKB:Q99878"
}